{
  "gene_symbol": "ANKRD20A3P",
  "term_id": "UNKNOWN:0001",
  "gene_name": "Putative ankyrin repeat domain-containing protein 20A3",
  "term_label": "Unknown molecular function",
  "gene": "UniProtKB:Q5VUR7"
}